{
  "gene": "UniProtKB:Q9UKR8",
  "term_id": "GO:0005886",
  "gene_name": "Tetraspanin-16",
  "gene_symbol": "TSPAN16",
  "term_label": "plasma membrane"
}